regulation of JNK cascade [GO:0046328] (biological process) Sources: GOC:bf Also known as: regulation of SAPK cascade Definition: Any process that modulates the frequency, rate or extent of signal transduction mediated by the JNK cascade. Subtypes: negative regulation of JNK cascade [GO:0046329], positive regulation of JNK cascade [GO:0046330] Relationships: is a type of regulation of MAPK cascade [GO:0043408]; regulates JNK cascade [GO:0007254]